thymine metabolic process [GO:0019859] (biological process) Also known as: thymine metabolism Relationships: is a type of pyrimidine nucleobase metabolic process [GO:0006206] Sources: GOC:go_curators Subtypes: thymine catabolic process [GO:0006210], thymine biosynthetic process [GO:0046106] Definition: The chemical reactions and pathways involving thymine, 5-methyluracil, one of the two major pyrimidine bases present (as thymidine) in DNA but not found in RNA other than (as ribothymidine) in transfer RNA, where it is a minor base.